tridecane metabolic process [GO:1900631] (biological process) Definition: The chemical reactions and pathways involving tridecane. Sources: GOC:TermGenie, GOC:mengo_curators Subtypes: tridecane biosynthetic process [GO:1900632] Also known as: tridecane metabolism Relationships: is a type of hydrocarbon metabolic process [GO:0120252]